{
  "term_label": "Unknown molecular function",
  "gene_symbol": "KLHDC8B",
  "term_id": "UNKNOWN:0001",
  "gene_name": "Kelch domain-containing protein 8B",
  "gene": "UniProtKB:Q8IXV7"
}